{
  "term_id": "GO:0007030",
  "gene_name": "Golgin-45",
  "gene_symbol": "BLZF1",
  "term_label": "Golgi organization",
  "gene": "UniProtKB:Q9H2G9"
}